{
  "term_label": "tRNA (m1A) methyltransferase complex",
  "gene": "UniProtKB:Q9BVS5",
  "gene_name": "tRNA (adenine(58)-N(1))-methyltransferase, mitochondrial",
  "term_id": "GO:0031515",
  "gene_symbol": "TRMT61B"
}